{
  "gene": "UniProtKB:A0A590UK83",
  "gene_name": "Small integral membrane protein 45",
  "term_id": "UNKNOWN:0001",
  "gene_symbol": "SMIM45",
  "term_label": "Unknown molecular function"
}